{
  "term_label": "Unknown cellular component",
  "gene_symbol": "DOK6",
  "term_id": "UNKNOWN:0003",
  "gene_name": "Docking protein 6",
  "gene": "UniProtKB:Q6PKX4"
}